{
  "gene_symbol": "DERPC",
  "gene": "UniProtKB:P0CG12",
  "gene_name": "Decreased expression in renal and prostate cancer protein",
  "term_label": "Unknown cellular component",
  "term_id": "UNKNOWN:0003"
}